{
  "gene_name": "Low-density lipoprotein receptor-related protein 8",
  "term_label": "ventral spinal cord development",
  "gene_symbol": "LRP8",
  "gene": "UniProtKB:Q14114",
  "term_id": "GO:0021517"
}